{
  "gene_name": "Glutaredoxin-like protein C5orf63",
  "term_id": "UNKNOWN:0001",
  "gene": "UniProtKB:A6NC05",
  "gene_symbol": "C5orf63",
  "term_label": "Unknown molecular function"
}